{
  "term_label": "Unknown molecular function",
  "gene_name": "Rab effector Noc2",
  "gene": "UniProtKB:Q9UNE2",
  "term_id": "UNKNOWN:0001",
  "gene_symbol": "RPH3AL"
}